islet amyloid polypeptide processing [GO:0034231] (biological process) Also known as: IAPP formation, IAPP processing, islet amyloid peptide formation, islet amyloid peptide processing, islet amyloid polypeptide formation Relationships: is a type of GO:0016486 Definition: The formation of mature islet amyloid polypeptide (IAPP) by posttranslational processing of pro-islet amyloid polypeptide (pro-IAPP). References: PMID:15983213, PMID:8262946 Sources: GOC:BHF, GOC:rl